DIM/DIP cell wall layer assembly [GO:0071770] (biological process) Definition: The aggregation, arrangement and bonding together of a set of components, including (phenyl)phthiocerol, phthiodiolone, phthiotriol dimycocerosate and diphthioceranate, to form the DIM/DIP layer of the Actinobacterium-type cell wall. Relationships: is a type of cellular component assembly [GO:0022607]; is part of Actinobacterium-type cell wall biogenesis [GO:0071766] References: PMID:15653820, PMID:3149973 Sources: GOC:mah, GOC:pr Also known as: DIM cell wall layer assembly, PDIM cell wall layer assembly, DIM/DIP cell wall layer biogenesis